{
  "gene_symbol": "CT45A8",
  "gene_name": "Cancer_testis antigen family 45 member A8",
  "term_id": "UNKNOWN:0003",
  "gene": "UniProtKB:P0DMV1",
  "term_label": "Unknown cellular component"
}